{
  "term_id": "GO:0016020",
  "gene": "UniProtKB:Q8TD20",
  "term_label": "membrane",
  "gene_name": "Solute carrier family 2, facilitated glucose transporter member 12",
  "gene_symbol": "SLC2A12"
}